{
  "term_label": "Unknown biological process",
  "gene_name": "G patch domain-containing protein 1",
  "gene_symbol": "GPATCH1",
  "gene": "UniProtKB:Q9BRR8",
  "term_id": "UNKNOWN:0002"
}